spongiotrophoblast differentiation [GO:0060708] (biological process) References: PMID:16269175 Sources: GOC:dph Also known as: spongiotrophoblast cell differentiation Definition: The process in which a relatively unspecialized cell of the ectoplacental cone acquires specialized features of a spongiotrophoblast of the placenta. A spongiotrophoblast cell is a basophilic cell. Relationships: is_a cell differentiation involved in embryonic placenta development [GO:0060706]; is part of spongiotrophoblast layer development [GO:0060712]